host chromosome [GO:0044383] (cellular component) Relationships: is a type of host intracellular organelle [GO:0033647] Sources: GOC:jl Definition: A structure composed of a very long molecule of DNA and associated proteins (e.g. histones) that carries hereditary information, occurring within a host cell.